{
  "gene_name": "Clathrin light chain B",
  "gene": "UniProtKB:P09497",
  "term_id": "GO:0030125",
  "gene_symbol": "CLTB",
  "term_label": "clathrin vesicle coat"
}